5-ureido-4-imidazole carboxylate hydrolase activity [GO:0043730] (molecular function) Relationships: is a type of hydrolase activity, acting on carbon-nitrogen (but not peptide) bonds, in linear amidines [GO:0016813] Definition: Catalysis of the reaction: 5-ureido-4-imidazole carboxylate + H2O = 5-amino-4-imidazole carboxylate + NH3 + CO2. Sources: GOC:jl